{
  "term_id": "GO:0005737",
  "gene_symbol": "OLA1",
  "term_label": "cytoplasm",
  "gene_name": "Obg-like ATPase 1",
  "gene": "UniProtKB:Q9NTK5"
}